L-methionine biosynthetic process from L-homoserine via O-acetyl-L-homoserine [GO:0019280] (BP) Definition: The chemical reactions and pathways resulting in the formation of methionine from L-homoserine, via the intermediate O-acetyl-L-homoserine using sulfur from hydrogen sulfide assimilation. Relationships: is a type of GO:0009092; is a type of L-methionine biosynthetic process [GO:0071265]; is a type of GO:0170041 Sources: GOC:go_curators, MetaCyc:HSERMETANA-PWY